{
  "term_label": "mannosyltransferase activity",
  "gene_name": "Protein O-mannosyl-transferase TMTC2",
  "gene": "UniProtKB:Q8N394",
  "gene_symbol": "TMTC2",
  "term_id": "GO:0000030"
}